{
  "gene_name": "Testis-expressed protein 38",
  "gene": "UniProtKB:Q6PEX7",
  "term_id": "UNKNOWN:0002",
  "term_label": "Unknown biological process",
  "gene_symbol": "TEX38"
}